{
  "gene": "UniProtKB:Q12857",
  "term_label": "regulation of transcription by RNA polymerase II",
  "gene_symbol": "NFIA",
  "term_id": "GO:0006357",
  "gene_name": "Nuclear factor 1 A-type"
}